{
  "term_id": "UNKNOWN:0002",
  "gene_name": "Divergent protein kinase domain 1B",
  "gene": "UniProtKB:Q5VUD6",
  "term_label": "Unknown biological process",
  "gene_symbol": "DIPK1B"
}